{
  "term_label": "Unknown biological process",
  "gene": "UniProtKB:Q8N6K0",
  "gene_name": "Testis-expressed protein 29",
  "term_id": "UNKNOWN:0002",
  "gene_symbol": "TEX29"
}